{
  "term_id": "UNKNOWN:0001",
  "gene_name": "Outer dense fiber protein 1",
  "term_label": "Unknown molecular function",
  "gene": "UniProtKB:Q14990",
  "gene_symbol": "ODF1"
}